vasculogenesis [GO:0001570] (biological process) References: PMID:8999798 Relationships: is a type of GO:0030154; is part of blood vessel morphogenesis [GO:0048514] Also known as: vascular morphogenesis Subtypes: central nervous system vasculogenesis [GO:0022009], GO:0060979 Regulation: regulated by regulation of vasculogenesis [GO:2001212]; negatively regulated by negative regulation of vasculogenesis [GO:2001213]; RO_0002213 by positive regulation of vasculogenesis [GO:2001214] Definition: The differentiation of endothelial cells from progenitor cells during blood vessel development, and the de novo formation of blood vessels and tubes.